myeloid leukocyte migration [GO:0097529] (biological process) References: PMID:22342843, PMID:24157461 Sources: GOC:cvs Definition: The movement of a myeloid leukocyte within or between different tissues and organs of the body. Relationships: is a type of GO:0050900 Subtypes: myeloid dendritic cell chemotaxis [GO:0002408], monocyte chemotaxis [GO:0002548], monocyte extravasation [GO:0035696], GO:0035703, granulocyte migration [GO:0097530], GO:0097531, macrophage migration [GO:1905517]